{
  "term_id": "GO:0003735",
  "gene_symbol": "RPS27A",
  "term_label": "structural constituent of ribosome",
  "gene": "UniProtKB:P62979",
  "gene_name": "Ubiquitin-ribosomal protein eS31 fusion protein"
}